{
  "gene": "UniProtKB:Q13156",
  "gene_name": "Replication protein A 30 kDa subunit",
  "gene_symbol": "RPA4",
  "term_label": "double-strand break repair via homologous recombination",
  "term_id": "GO:0000724"
}